{
  "gene_name": "Putative insulin-like growth factor 2 antisense gene protein",
  "term_label": "Unknown cellular component",
  "gene": "UniProtKB:Q6U949",
  "term_id": "UNKNOWN:0003",
  "gene_symbol": "IGF2-AS"
}